{
  "gene_symbol": "GNLY",
  "term_label": "Unknown molecular function",
  "gene": "UniProtKB:P22749",
  "gene_name": "Granulysin",
  "term_id": "UNKNOWN:0001"
}